{
  "gene": "UniProtKB:Q9BXI2",
  "gene_name": "Mitochondrial ornithine transporter 2",
  "term_label": "mitochondrial L-ornithine transmembrane transport",
  "gene_symbol": "SLC25A2",
  "term_id": "GO:1990575"
}